{
  "gene": "UniProtKB:A8MZH6",
  "term_label": "Unknown biological process",
  "gene_symbol": "OOSP1",
  "term_id": "UNKNOWN:0002",
  "gene_name": "Putative oocyte-secreted protein 1 homolog"
}